{
  "gene_symbol": "NPAP1",
  "gene": "UniProtKB:Q9NZP6",
  "term_label": "structural constituent of nuclear pore",
  "gene_name": "Nuclear pore-associated protein 1",
  "term_id": "GO:0017056"
}